{
  "gene_symbol": "RELB",
  "gene": "UniProtKB:Q01201",
  "gene_name": "Transcription factor RelB",
  "term_id": "GO:0034097",
  "term_label": "response to cytokine"
}